{
  "term_id": "GO:0006357",
  "gene": "UniProtKB:Q15744",
  "gene_symbol": "CEBPE",
  "term_label": "regulation of transcription by RNA polymerase II",
  "gene_name": "CCAAT_enhancer-binding protein epsilon"
}